{
  "gene": "UniProtKB:Q9H8H3",
  "term_id": "UNKNOWN:0003",
  "gene_symbol": "TMT1A",
  "gene_name": "N6-adenosine-methyltransferase TMT1A",
  "term_label": "Unknown cellular component"
}